dynein intermediate chain binding [GO:0045505] (molecular function) Definition: Binding to an intermediate chain of the dynein complex. Sources: GOC:bf Relationships: is a type of protein binding [GO:0005515]